{
  "term_id": "GO:0000139",
  "gene_name": "Probable UDP-sugar transporter protein SLC35A5",
  "term_label": "Golgi membrane",
  "gene": "UniProtKB:Q9BS91",
  "gene_symbol": "SLC35A5"
}